amidinotransferase activity [GO:0015067] (molecular function) Subtypes: glycine amidinotransferase activity [GO:0015068], scyllo-inosamine-4-phosphate amidinotransferase activity [GO:0015069] Definition: Catalysis of the reversible transfer of an amidino group to an acceptor. Also known as: transamidinase activity Relationships: is a type of GO:0016741 Sources: GOC:ai